neuron spine [GO:0044309] (CC) Subtypes: dendritic spine [GO:0043197], GO:0044308, somatic spine [GO:0097465] Sources: ISBN:0198504888, NIF_Subcellular:sao1145756102 Relationships: is a type of neuron projection [GO:0043005] Also known as: spine Definition: A small membranous protrusion, often ending in a bulbous head and attached to the neuron by a narrow stalk or neck.